{
  "gene": "UniProtKB:Q9Y6I9",
  "term_id": "GO:0005657",
  "term_label": "replication fork",
  "gene_name": "Testis-expressed protein 264",
  "gene_symbol": "TEX264"
}